{
  "gene_symbol": "FLT4",
  "gene_name": "Vascular endothelial growth factor receptor 3",
  "term_id": "GO:0005886",
  "term_label": "plasma membrane",
  "gene": "UniProtKB:P35916"
}